{
  "gene_name": "Zinc finger protein 576",
  "gene_symbol": "ZNF576",
  "term_id": "UNKNOWN:0002",
  "gene": "UniProtKB:Q9H609",
  "term_label": "Unknown biological process"
}